{
  "gene": "UniProtKB:P08684",
  "gene_symbol": "CYP3A4",
  "term_label": "testosterone 6-beta-hydroxylase activity",
  "gene_name": "Cytochrome P450 3A4",
  "term_id": "GO:0050649"
}